{
  "gene_symbol": "KIAA1217",
  "gene_name": "Sickle tail protein homolog",
  "term_id": "UNKNOWN:0001",
  "term_label": "Unknown molecular function",
  "gene": "UniProtKB:Q5T5P2"
}